{
  "gene_name": "PRKCA-binding protein",
  "gene_symbol": "PICK1",
  "term_id": "GO:0005080",
  "term_label": "protein kinase C binding",
  "gene": "UniProtKB:Q9NRD5"
}